regulation of phosphorylation [GO:0042325] (biological process) Note: Note that this term is in the subset of terms that should not be used for direct gene product annotation. Instead, select a child term or, if no appropriate child term exists, please request a new term. Direct annotations to this term may be amended during annotation QC. Subtypes: regulation of protein phosphorylation [GO:0001932], negative regulation of phosphorylation [GO:0042326], positive regulation of phosphorylation [GO:0042327], regulation of kinase activity [GO:0043549] Sources: GOC:jl Definition: Any process that modulates the frequency, rate or extent of addition of phosphate groups into a molecule. Relationships: is a type of GO:0051174; regulates GO:0016310